{
  "gene": "UniProtKB:A6NFH5",
  "gene_name": "Fatty acid-binding protein 12",
  "gene_symbol": "FABP12",
  "term_id": "GO:0005504",
  "term_label": "fatty acid binding"
}